coated vesicle [GO:0030135] (cellular component) Relationships: is a type of cytoplasmic vesicle [GO:0031410] Definition: Small membrane-bounded organelle formed by pinching off of a coated region of membrane. Some coats are made of clathrin, whereas others are made from other proteins. Subtypes: COPII-coated ER to Golgi transport vesicle [GO:0030134], GO:0030136, COPI-coated vesicle [GO:0030137] Sources: ISBN:0815316194